SCF-Skp2 ubiquitin ligase complex [GO:0097669] (cellular component) Definition: An SCF ubiquitin ligase complex in which the F-box protein is Skp2 in S. cerevisiae. References: PMID:14747994 Sources: GOC:jd, GOC:vw Relationships: is a type of GO:0019005